{
  "term_id": "UNKNOWN:0002",
  "term_label": "Unknown biological process",
  "gene": "UniProtKB:Q9BV87",
  "gene_symbol": "CNPPD1",
  "gene_name": "Protein CNPPD1"
}